{
  "gene_name": "Integrin alpha-X",
  "gene": "UniProtKB:P20702",
  "gene_symbol": "ITGAX",
  "term_id": "GO:0038023",
  "term_label": "signaling receptor activity"
}